{
  "gene_name": "Interleukin-24",
  "gene_symbol": "IL24",
  "term_label": "extracellular space",
  "gene": "UniProtKB:Q13007",
  "term_id": "GO:0005615"
}